{
  "gene_symbol": "THAP11",
  "term_label": "nucleoplasm",
  "gene": "UniProtKB:Q96EK4",
  "term_id": "GO:0005654",
  "gene_name": "THAP domain-containing protein 11"
}